{
  "gene": "UniProtKB:Q96IZ0",
  "gene_name": "PRKC apoptosis WT1 regulator protein",
  "term_label": "positive regulation of neuron apoptotic process",
  "term_id": "GO:0043525",
  "gene_symbol": "PAWR"
}